{
  "term_label": "endocytic recycling",
  "gene": "UniProtKB:Q9H0T7",
  "gene_name": "Ras-related protein Rab-17",
  "term_id": "GO:0032456",
  "gene_symbol": "RAB17"
}